{
  "gene_name": "Extracellular superoxide dismutase [Cu-Zn]",
  "gene_symbol": "SOD3",
  "term_label": "copper ion binding",
  "term_id": "GO:0005507",
  "gene": "UniProtKB:P08294"
}